{
  "gene_symbol": "UCN3",
  "term_id": "GO:0005615",
  "gene_name": "Urocortin-3",
  "gene": "UniProtKB:Q969E3",
  "term_label": "extracellular space"
}